{
  "gene_symbol": "DENND4A",
  "term_id": "GO:0005085",
  "term_label": "guanyl-nucleotide exchange factor activity",
  "gene_name": "C-myc promoter-binding protein",
  "gene": "UniProtKB:Q7Z401"
}